{
  "gene_name": "Protein FAM118B",
  "gene_symbol": "FAM118B",
  "term_id": "UNKNOWN:0002",
  "term_label": "Unknown biological process",
  "gene": "UniProtKB:Q9BPY3"
}